positive regulation of protein localization to centrosome [GO:1904781] (biological process) Also known as: positive regulation of protein localisation to centrosome, up regulation of protein localisation to centrosome, up regulation of protein localization to centrosome, up-regulation of protein localisation to centrosome, up-regulation of protein localization to centrosome, upregulation of protein localisation to centrosome, upregulation of protein localization to centrosome, activation of protein localisation to centrosome, activation of protein localization to centrosome Note: An example is cdk-2 in C. elegans (UniProt ID O61847) in PMID:17115027 (inferred from mutant phenotype). Definition: Any process that activates or increases the frequency, rate or extent of protein localization to centrosome. Relationships: is a type of positive regulation of protein localization [GO:1903829]; is a type of GO:1904779; positively regulates protein localization to centrosome [GO:0071539] References: PMID:17115027 Sources: GOC:TermGenie, GO_REF:0000058